{
  "term_label": "intracellular signal transduction",
  "gene": "UniProtKB:Q5KSL6",
  "gene_symbol": "DGKK",
  "term_id": "GO:0035556",
  "gene_name": "Diacylglycerol kinase kappa"
}